{
  "gene_name": "Kinesin-like protein KIF1B",
  "gene_symbol": "KIF1B",
  "gene": "UniProtKB:O60333",
  "term_label": "retrograde neuronal dense core vesicle transport",
  "term_id": "GO:1990049"
}